intramolecular oxidoreductase activity, transposing C=C bonds [GO:0016863] (molecular function) Also known as: intramolecular isomerase activity, transposing C=C bonds Definition: Catalysis of an oxidation-reduction (redox) reaction in which the hydrogen donor and acceptor are the same molecule, one or more carbon-carbon double bonds in the molecule are rearranged, and no oxidized product appears. Sources: EC:5.3.3.-, GOC:mah Subtypes: C-8 sterol isomerase activity [GO:0000247], delta(3)-delta(2)-enoyl-CoA isomerase activity [GO:0004165], dopachrome isomerase activity [GO:0004167], isopentenyl-diphosphate delta-isomerase activity [GO:0004452], steroid Delta-isomerase activity [GO:0004769], 5-carboxymethyl-2-hydroxymuconate delta-isomerase activity [GO:0008704], muconolactone delta-isomerase activity [GO:0016159], polyenoic fatty acid isomerase activity [GO:0034016], trans-2-decenoyl-acyl-carrier-protein isomerase activity [GO:0034017], aconitate delta-isomerase activity [GO:0047614], cholestenol delta-isomerase activity [GO:0047750], isopiperitenone delta-isomerase activity [GO:0050008], methylitaconate delta-isomerase activity [GO:0050100], GO:0050219, vinylacetyl-CoA delta-isomerase activity [GO:0050393], GO:0051750, trans-2,3-dihydro-3-hydroxy-anthranilate isomerase activity [GO:0102943], dopaminechrome tautomerase activity [GO:0106417] Relationships: is_a intramolecular oxidoreductase activity [GO:0016860]